establishment or maintenance of cell polarity [GO:0007163] (biological process) Also known as: cell polarity, establishment and/or maintenance of cell polarity, establishment and/or maintenance of cell polarization Subtypes: GO:0016332, establishment or maintenance of polarity of follicular epithelium [GO:0016334], establishment or maintenance of polarity of larval imaginal disc epithelium [GO:0016336], establishment of cell polarity [GO:0030010], maintenance of cell polarity [GO:0030011], establishment or maintenance of cytoskeleton polarity [GO:0030952], GO:0042067, establishment or maintenance of neuroblast polarity [GO:0045196], establishment or maintenance of bipolar cell polarity [GO:0061245], establishment or maintenance of monopolar cell polarity [GO:0061339], establishment or maintenance of cell polarity regulating cell shape [GO:0071963] Relationships: is_a GO:0009987 Regulation: regulated by GO:0032878 Sources: GOC:mah Definition: Any cellular process that results in the specification, formation or maintenance of anisotropic intracellular organization or cell growth patterns.